regulation of tRNA C5-cytosine methylation [GO:0110003] (biological process) Subtypes: GO:0110005 References: PMID:23074192 Sources: GOC:vw Definition: Any process that modulates the frequency, rate or extent of the chemical reactions and pathways involving tRNA C5-cytosine methylation. Relationships: is a type of regulation of tRNA methylation [GO:0110002]; regulates tRNA C5-cytosine methylation [GO:0002946]